NuA3b histone acetyltransferase complex [GO:1990468] (cellular component) Relationships: is a type of NuA3 histone acetyltransferase complex [GO:0033100] References: PMID:25104842 Sources: GOC:rb Definition: A NuA3 complex that catalyzes the acetylation of Histone H3. In S. cerevisiae, this complex consists of Eaf6p, Nto1p, Sas3p, Taf14p, Pdp3 and associates with H3K4me3 via Pdp3p.